rRNA (pseudouridine) methyltransferase activity [GO:0070037] (molecular function) Definition: Catalysis of the transfer of a methyl group from S-adenosyl-L-methionine to a pseudouridine residue in an rRNA molecule. Sources: GOC:imk, GOC:mah Relationships: is a type of rRNA methyltransferase activity [GO:0008649] Subtypes: GO:0070038